{
  "gene_name": "Elongation of very long chain fatty acids protein 6",
  "gene": "UniProtKB:Q9H5J4",
  "gene_symbol": "ELOVL6",
  "term_label": "very long-chain fatty acid biosynthetic process",
  "term_id": "GO:0042761"
}